3-alpha-hydroxycholanate dehydrogenase activity [GO:0047043] (molecular function) Sources: EC:1.1.1.52, RHEA:19585 Also known as: 3alpha-hydroxy-5beta-cholanate:NAD+ oxidoreductase activity, 3alpha-hydroxycholanate dehydrogenase activity, alpha-hydroxy-cholanate dehydrogenase activity Definition: Catalysis of the reaction: lithocholate + NAD+ = 3-oxo-5beta-cholanate + H+ + NADH. Relationships: is a type of oxidoreductase activity, acting on the CH-OH group of donors, NAD or NADP as acceptor [GO:0016616]